{
  "gene": "UniProtKB:Q6ZSR9",
  "term_label": "Unknown cellular component",
  "term_id": "UNKNOWN:0003",
  "gene_name": "Uncharacterized protein FLJ45252",
  "gene_symbol": "Q6ZSR9"
}